{
  "gene_name": "Eukaryotic translation initiation factor 3 subunit C-like protein",
  "gene_symbol": "EIF3CL",
  "gene": "UniProtKB:B5ME19",
  "term_id": "GO:0006413",
  "term_label": "translational initiation"
}